{
  "term_id": "GO:0007173",
  "gene_name": "Tyrosine-protein kinase ABL2",
  "gene_symbol": "ABL2",
  "gene": "UniProtKB:P42684",
  "term_label": "epidermal growth factor receptor signaling pathway"
}